{
  "term_label": "Unknown molecular function",
  "gene_name": "Reticulophagy regulator 2",
  "term_id": "UNKNOWN:0001",
  "gene_symbol": "RETREG2",
  "gene": "UniProtKB:Q8NC44"
}